{
  "term_id": "UNKNOWN:0002",
  "gene": "UniProtKB:Q8NA69",
  "gene_name": "Testis-expressed protein 45",
  "term_label": "Unknown biological process",
  "gene_symbol": "TEX45"
}